{
  "gene_name": "Serpin B4",
  "term_id": "UNKNOWN:0002",
  "gene_symbol": "SERPINB4",
  "term_label": "Unknown biological process",
  "gene": "UniProtKB:P48594"
}